striatum development [GO:0021756] (biological process) Definition: The progression of the striatum over time from its initial formation until its mature state. The striatum is a region of the forebrain consisting of the caudate nucleus, putamen and fundus striati. Sources: GOC:cls, GOC:dgh, GOC:dph, GOC:jid, GO_REF:0000021 Also known as: neostriatum development, striate nucleus development Relationships: is a type of anatomical structure development [GO:0048856]; is part of subpallium development [GO:0021544]